{
  "term_label": "tRNA dihydrouridine synthase activity",
  "gene": "UniProtKB:Q9NX74",
  "term_id": "GO:0017150",
  "gene_name": "tRNA-dihydrouridine(20) synthase [NAD(P)+]-like",
  "gene_symbol": "DUS2"
}